{
  "gene_symbol": "NR1D2",
  "term_label": "intracellular receptor signaling pathway",
  "gene": "UniProtKB:Q14995",
  "gene_name": "Nuclear receptor subfamily 1 group D member 2",
  "term_id": "GO:0030522"
}